anticlinal cell division [GO:0090510] (biological process) References: PMID:21391814 Sources: GOC:tair_curators Definition: A cell division process where the division plane is perpendicular to the surface of the organ. It adds cells to the existing cell layer or cell file. Relationships: is a type of cell division [GO:0051301]